{
  "gene": "UniProtKB:P12081",
  "term_label": "RNA binding",
  "gene_symbol": "HARS1",
  "term_id": "GO:0003723",
  "gene_name": "Histidine--tRNA ligase, cytoplasmic"
}